sensory perception of slow pain [GO:0019235] (BP) Definition: The series of events required for an organism to receive a slow pain stimulus, convert it to a molecular signal, and recognize and characterize the signal. This is a neurological process. Slow pain is often subjectively described as an aching or throbbing pain; in humans, the signals from a slow pain stimulus are perceived and relayed along unmyelinated C fibers to the central nervous system, reaching their target in about 1 second. Slow pain is often associated with tissue destruction. References: PMID:38704307 Sources: http://www.people.vcu.edu/~mikuleck/ssspain/ Relationships: is a type of sensory perception of pain [GO:0019233]